{
  "gene": "UniProtKB:Q6UXY8",
  "term_id": "UNKNOWN:0003",
  "gene_name": "Transmembrane channel-like protein 5",
  "gene_symbol": "TMC5",
  "term_label": "Unknown cellular component"
}